{
  "gene_name": "Protein PAXX",
  "gene": "UniProtKB:Q9BUH6",
  "gene_symbol": "PAXX",
  "term_label": "site of double-strand break",
  "term_id": "GO:0035861"
}